{
  "gene": "UniProtKB:Q8N5M1",
  "gene_symbol": "ATPAF2",
  "term_id": "GO:0033615",
  "term_label": "mitochondrial proton-transporting ATP synthase complex assembly",
  "gene_name": "ATP synthase mitochondrial F1 complex assembly factor 2"
}